interleukin-12 receptor binding [GO:0005143] (molecular function) Relationships: is a type of cytokine receptor binding [GO:0005126]; is a type of growth factor receptor binding [GO:0070851] Sources: GOC:ai Definition: Binding to an interleukin-12 receptor. Also known as: IL-12, interleukin-12 receptor ligand